regulation of anterograde synaptic vesicle transport [GO:1903742] (biological process) Relationships: is a type of regulation of vesicle transport along microtubule [GO:1901608]; is a type of GO:1902803; regulates anterograde synaptic vesicle transport [GO:0048490] References: PMID:25329901 Sources: GOC:TermGenie, GOC:kmv, GO_REF:0000058 Definition: Any process that modulates the frequency, rate or extent of anterograde synaptic vesicle transport. Subtypes: GO:1903743, GO:1903744